endoplasmic reticulum-Golgi intermediate compartment (ERGIC) derived vesicle fusion with endoplasmic reticulum membrane [GO:1990669] (biological process) Relationships: is a type of vesicle fusion with endoplasmic reticulum [GO:0048279]; is part of retrograde vesicle-mediated transport, Golgi to endoplasmic reticulum [GO:0006890] References: PMID:16038056, PMID:24119662 Sources: GOC:bhm Definition: The joining of the lipid bilayer membrane around an ERGIC-derived vesicle to the lipid bilayer membrane of the ER. Such vesicles include COPI-coated transport vesicles involved in retrograde transport. Also known as: ER-Golgi intermediate compartment derived vesicle fusion with ER membrane, endoplasmic reticulum-Golgi intermediate compartment (ERGIC) derived vesicle fusion with ER membrane